SNARE complex assembly [GO:0035493] (BP) References: PMID:10872468 Sources: GOC:rb Relationships: is a type of protein-containing complex assembly [GO:0065003]; is part of GO:0006906 Definition: The aggregation, arrangement and bonding together of a set of components to form a SNARE complex, a protein complex involved in membrane fusion; a stable ternary complex consisting of a four-helix bundle, usually formed from one R-SNARE and three Q-SNAREs with an ionic layer sandwiched between hydrophobic layers. Regulation: regulated by regulation of SNARE complex assembly [GO:0035542]; positively regulated by positive regulation of SNARE complex assembly [GO:0035543]; negatively regulated by GO:0035544